{
  "gene_symbol": "LIMCH1",
  "gene": "UniProtKB:Q9UPQ0",
  "gene_name": "LIM and calponin homology domains-containing protein 1",
  "term_label": "stress fiber",
  "term_id": "GO:0001725"
}